{
  "term_label": "plasma membrane tubulation",
  "term_id": "GO:0097320",
  "gene_name": "Sorting nexin-33",
  "gene": "UniProtKB:Q8WV41",
  "gene_symbol": "SNX33"
}